{
  "gene_symbol": "GTF2H3",
  "gene_name": "General transcription factor IIH subunit 3",
  "term_id": "GO:0016251",
  "gene": "UniProtKB:Q13889",
  "term_label": "RNA polymerase II general transcription initiation factor activity"
}